serine 2-dehydrogenase activity [GO:0050282] (molecular function) Definition: Catalysis of the reaction: L-serine + H2O + NAD+ = 3-hydroxypyruvate + NH3 + NADH. Sources: EC:1.4.1.7, MetaCyc:SERINE-DEHYDROGENASE-RXN Also known as: serine dehydrogenase activity, L-serine:NAD oxidoreductase (deaminating) activity, L-serine:NAD+ 2-oxidoreductase (deaminating) Relationships: is a type of GO:0016639